{
  "gene_symbol": "C17orf107",
  "term_id": "UNKNOWN:0001",
  "gene": "UniProtKB:Q6ZR85",
  "term_label": "Unknown molecular function",
  "gene_name": "Uncharacterized protein C17orf107"
}